slug development involved in sorocarp development [GO:0031153] (biological process) Also known as: pseudoplasmodium biosynthesis, pseudoplasmodium formation, slug development during fruiting body development, migratory slug development during sorocarp development, standing slug development during sorocarp development, slug development during sorocarp development Relationships: is a type of socially cooperative development [GO:0099120]; is part of GO:0030587 Sources: GOC:mah, GOC:mtg_sensu, ISBN:0521583640 Definition: The process whose specific outcome is the progression of the slug over time, from its formation to the mature structure. Slug development begins when the aggregate rises upwards to form a finger-shaped structure and ends when culmination begins. Slug development begins after aggregation and ends before culmination in sorocarp development.